structural constituent of chitin-based cuticle [GO:0005214] (molecular function) Sources: GOC:mah, GOC:mtg_sensu Definition: The action of a molecule that contributes to the structural integrity of a chitin-based cuticle. An example of this is found in Drosophila melanogaster. Relationships: is a type of structural constituent of cuticle [GO:0042302] Subtypes: structural constituent of chitin-based larval cuticle [GO:0008010], structural constituent of pupal chitin-based cuticle [GO:0008011], structural constituent of adult chitin-based cuticle [GO:0008012]